{
  "term_id": "GO:0000978",
  "term_label": "RNA polymerase II cis-regulatory region sequence-specific DNA binding",
  "gene_name": "Putative zinc finger protein 137",
  "gene_symbol": "ZNF137P",
  "gene": "UniProtKB:P52743"
}